conversion of O-phosphoseryl-tRNA to cysteinyl-tRNA [GO:0071952] (biological process) References: PMID:17351629, PMID:18559341 Sources: GOC:jsg Note: Note that this process has been observed in some archaeal and bacterial species. Definition: The modification process that results in the conversion of O-phosphoserine charged on a tRNA(Cys) to cysteinyl-tRNA. Relationships: is a type of charged-tRNA amino acid modification [GO:0019988]